positive regulation of cell cycle [GO:0045787] (biological process) Also known as: positive regulation of cell cycle progression, positive regulation of progression through cell cycle, up regulation of progression through cell cycle, up-regulation of progression through cell cycle, upregulation of progression through cell cycle, activation of progression through cell cycle, stimulation of progression through cell cycle Definition: Any process that activates or increases the rate or extent of progression through the cell cycle. Relationships: is_a positive regulation of cellular process [GO:0048522]; is a type of regulation of cell cycle [GO:0051726]; RO_0002213 GO:0007049 Sources: GOC:go_curators Subtypes: positive regulation of cyclin-dependent protein serine/threonine kinase activity [GO:0045737], positive regulation of mitotic cell cycle [GO:0045931], positive regulation of meiotic cell cycle [GO:0051446], positive regulation of cell cycle process [GO:0090068]